{
  "term_id": "GO:0006357",
  "gene_symbol": "POU6F2",
  "term_label": "regulation of transcription by RNA polymerase II",
  "gene": "UniProtKB:P78424",
  "gene_name": "POU domain, class 6, transcription factor 2"
}